{
  "term_id": "GO:0005813",
  "gene": "UniProtKB:Q13432",
  "term_label": "centrosome",
  "gene_symbol": "UNC119",
  "gene_name": "Protein unc-119 homolog A"
}